{
  "gene_name": "Transcription factor EB",
  "term_id": "GO:0000978",
  "term_label": "RNA polymerase II cis-regulatory region sequence-specific DNA binding",
  "gene": "UniProtKB:P19484",
  "gene_symbol": "TFEB"
}